{
  "term_label": "membrane",
  "gene": "UniProtKB:Q8N357",
  "gene_symbol": "SLC35F6",
  "gene_name": "Solute carrier family 35 member F6",
  "term_id": "GO:0016020"
}